{
  "term_id": "GO:0005886",
  "term_label": "plasma membrane",
  "gene_symbol": "GPR139",
  "gene": "UniProtKB:Q6DWJ6",
  "gene_name": "Probable G-protein coupled receptor 139"
}